{
  "gene_name": "Beta-crystallin B1",
  "gene_symbol": "CRYBB1",
  "term_label": "lens development in camera-type eye",
  "term_id": "GO:0002088",
  "gene": "UniProtKB:P53674"
}